{
  "term_label": "RAVE complex",
  "gene_name": "Protein rogdi homolog",
  "gene": "UniProtKB:Q9GZN7",
  "term_id": "GO:0043291",
  "gene_symbol": "ROGDI"
}